striated muscle cell development [GO:0055002] (biological process) Definition: The process whose specific outcome is the progression of a striated muscle cell over time, from its formation to the mature structure. Striated muscle cells contain fibers that are divided by transverse bands into striations, and cardiac and skeletal muscle are types of striated muscle. Sources: CL:0000737, GOC:devbiol Relationships: is a type of muscle cell development [GO:0055001]; is part of striated muscle cell differentiation [GO:0051146] Subtypes: GO:0014904, cardiac muscle cell development [GO:0055013]